{
  "gene_name": "Prokineticin receptor 1",
  "gene_symbol": "PROKR1",
  "gene": "UniProtKB:Q8TCW9",
  "term_id": "GO:0007186",
  "term_label": "G protein-coupled receptor signaling pathway"
}